{
  "gene": "UniProtKB:O60258",
  "gene_name": "Fibroblast growth factor 17",
  "term_label": "neurogenesis",
  "gene_symbol": "FGF17",
  "term_id": "GO:0022008"
}